{
  "term_id": "GO:0005737",
  "gene": "UniProtKB:P21291",
  "term_label": "cytoplasm",
  "gene_symbol": "CSRP1",
  "gene_name": "Cysteine and glycine-rich protein 1"
}